phosphatase activator activity [GO:0019211] (molecular function) Sources: GOC:ai Relationships: is a type of enzyme activator activity [GO:0008047]; is a type of phosphatase regulator activity [GO:0019208]; positively regulates phosphatase activity [GO:0016791] Subtypes: protein phosphatase activator activity [GO:0072542] Definition: Binds to and increases the activity of a phosphatase.